{
  "term_id": "GO:0005765",
  "term_label": "lysosomal membrane",
  "gene_name": "HLA class II histocompatibility antigen, DR beta 4 chain",
  "gene": "UniProtKB:P13762",
  "gene_symbol": "HLA-DRB4"
}